tetrahydromethanopterin S-methyltransferase activity [GO:0030269] (molecular function) Definition: Catalysis of the reaction: 5-methyl-5,6,7,8-tetrahydromethanopterin + coenzyme M + 2 Na+(in) = 5,6,7,8-tetrahydromethanopterin + methyl-coenzyme M + 2 Na+(out). 2-(methylthio)ethanesulfonate is also known as methyl-CoM. Sources: RHEA:53492 Also known as: 5-methyl-5,6,7,8-tetrahydromethanopterin:2-mercaptoethanesulfonate 2-methyltransferase activity, N(5)-methyltetrahydromethanopterin--coenzyme M methyltransferase activity, N5-methyltetrahydromethanopterin--coenzyme M methyltransferase activity, tetrahydromethanopterin methyltransferase activity Relationships: is a type of S-methyltransferase activity [GO:0008172]; is a type of sodium ion transmembrane transporter activity [GO:0015081]; is a type of 5-methyl-5,6,7,8-tetrahydromethanopterin-dependent methyltransferase activity [GO:0042086]